{
  "gene": "UniProtKB:P18146",
  "gene_name": "Early growth response protein 1",
  "term_id": "GO:0006357",
  "gene_symbol": "EGR1",
  "term_label": "regulation of transcription by RNA polymerase II"
}